{
  "gene": "UniProtKB:Q8WZ26",
  "gene_symbol": "PP6455",
  "term_id": "UNKNOWN:0002",
  "term_label": "Unknown biological process",
  "gene_name": "Putative uncharacterized protein PP6455"
}